{
  "term_id": "GO:0032979",
  "gene_symbol": "MAIP1",
  "gene": "UniProtKB:Q8WWC4",
  "term_label": "protein insertion into mitochondrial inner membrane from matrix",
  "gene_name": "m-AAA protease-interacting protein 1, mitochondrial"
}